{
  "gene_name": "E3 ubiquitin-protein ligase RNF217",
  "term_label": "cytoplasm",
  "gene": "UniProtKB:Q8TC41",
  "term_id": "GO:0005737",
  "gene_symbol": "RNF217"
}